{
  "gene_name": "Small nuclear ribonucleoprotein-associated proteins B and B'",
  "gene_symbol": "SNRPB",
  "term_label": "U2-type prespliceosome",
  "gene": "UniProtKB:P14678",
  "term_id": "GO:0071004"
}